{
  "gene": "UniProtKB:Q99593",
  "gene_name": "T-box transcription factor TBX5",
  "term_id": "GO:0000981",
  "gene_symbol": "TBX5",
  "term_label": "DNA-binding transcription factor activity, RNA polymerase II-specific"
}